11-deoxycortisol binding [GO:1903876] (molecular function) Definition: Binding to 11-deoxycortisol. References: PMID:10802282 Sources: GOC:TermGenie, GO_REF:0000067 Relationships: is a type of GO:0043178; is a type of steroid hormone binding [GO:1990239]